{
  "term_label": "oxidoreductase activity",
  "term_id": "GO:0016491",
  "gene_symbol": "CYGB",
  "gene": "UniProtKB:Q8WWM9",
  "gene_name": "Cytoglobin"
}